{
  "gene": "UniProtKB:O75676",
  "term_id": "GO:0005654",
  "gene_name": "Ribosomal protein S6 kinase alpha-4",
  "gene_symbol": "RPS6KA4",
  "term_label": "nucleoplasm"
}